{
  "gene_symbol": "GRIFIN",
  "term_id": "GO:0030246",
  "term_label": "carbohydrate binding",
  "gene": "UniProtKB:A4D1Z8",
  "gene_name": "Grifin"
}